{
  "term_label": "DNA-binding transcription factor activity, RNA polymerase II-specific",
  "gene_name": "Myoneurin",
  "gene_symbol": "MYNN",
  "term_id": "GO:0000981",
  "gene": "UniProtKB:Q9NPC7"
}